cyclopentanol biosynthetic process [GO:0033021] (biological process) References: PMID:12406764 Sources: GOC:mah Also known as: cyclopentanol anabolism, cyclopentanol biosynthesis, cyclopentanol formation, cyclopentanol synthesis Relationships: is a type of alcohol biosynthetic process [GO:0046165] Definition: The chemical reactions and pathways resulting in the formation of cyclopentanol.